polyphenic determination, influence by environmental factors [GO:0048651] (biological process) Definition: The process in which individuals that have the potential to develop any of several possible distinct developmental paths have their individual developmental fates determined in response to environmental cues. Subtypes: caste determination, influence by environmental factors [GO:0048650] Relationships: is a type of response to external stimulus [GO:0009605]; is a type of polyphenic determination [GO:0048647] Sources: GOC:jid